regulation of hydrogen peroxide metabolic process [GO:0010310] (biological process) References: PMID:14765119 Definition: Any process that modulates the frequency, rate or extent of the chemical reactions and pathways involving hydrogen peroxide. Relationships: is_a regulation of reactive oxygen species metabolic process [GO:2000377]; regulates hydrogen peroxide metabolic process [GO:0042743] Also known as: regulation of hydrogen peroxide metabolism Subtypes: negative regulation of hydrogen peroxide metabolic process [GO:0010727], regulation of hydrogen peroxide biosynthetic process [GO:0010728], regulation of hydrogen peroxide catabolic process [GO:2000295]